{
  "gene_symbol": "ZNF722",
  "gene_name": "Zinc finger protein 722",
  "term_label": "DNA-binding transcription factor activity, RNA polymerase II-specific",
  "term_id": "GO:0000981",
  "gene": "UniProtKB:A0A1W2PQL4"
}